sabinene-hydrate synthase activity [GO:0050469] (MF) Also known as: geranyl-diphosphate diphosphate-lyase (cyclizing, sabinene-hydrate-forming), sabinene hydrate cyclase activity Definition: Catalysis of the reaction: geranyl diphosphate + H2O = diphosphate + sabinene hydrate. Relationships: is a type of carbon-oxygen lyase activity, acting on phosphates [GO:0016838] Sources: EC:4.2.3.11, RHEA:19565